rhamnogalacturonan I side chain metabolic process [GO:0010400] (biological process) Sources: GOC:tair_curators Relationships: is a type of GO:0010395 Definition: The chemical reactions and pathways involving the side chains of the pectin, rhamnogalacturonan I. Also known as: rhamnogalacturonan I side chain metabolism Subtypes: pectic galactan metabolic process [GO:0010401]